{
  "term_id": "UNKNOWN:0003",
  "gene_name": "Zinc finger protein 511",
  "gene": "UniProtKB:Q8NB15",
  "term_label": "Unknown cellular component",
  "gene_symbol": "ZNF511"
}